{
  "gene": "UniProtKB:A0A1B0GTI1",
  "term_id": "UNKNOWN:0003",
  "gene_name": "Coiled-coil domain-containing protein 201",
  "gene_symbol": "CCDC201",
  "term_label": "Unknown cellular component"
}